{
  "gene": "UniProtKB:Q15573",
  "term_id": "UNKNOWN:0002",
  "term_label": "Unknown biological process",
  "gene_symbol": "TAF1A",
  "gene_name": "TATA box-binding protein-associated factor RNA polymerase I subunit A"
}